{
  "gene": "UniProtKB:Q15555",
  "gene_name": "Microtubule-associated protein RP_EB family member 2",
  "gene_symbol": "MAPRE2",
  "term_id": "GO:0035371",
  "term_label": "microtubule plus-end"
}